{
  "gene": "UniProtKB:Q96PS6",
  "gene_symbol": "GAFA1",
  "gene_name": "Putative uncharacterized protein GAFA-1",
  "term_id": "UNKNOWN:0001",
  "term_label": "Unknown molecular function"
}